{
  "gene_symbol": "RPL27A",
  "term_id": "UNKNOWN:0002",
  "gene": "UniProtKB:P46776",
  "term_label": "Unknown biological process",
  "gene_name": "Large ribosomal subunit protein uL15"
}